{
  "gene": "UniProtKB:Q9H9T3",
  "term_id": "GO:0005737",
  "gene_name": "Elongator complex protein 3",
  "term_label": "cytoplasm",
  "gene_symbol": "ELP3"
}